{
  "gene_symbol": "SPEF1",
  "gene": "UniProtKB:Q9Y4P9",
  "term_label": "microtubule binding",
  "gene_name": "Sperm flagellar protein 1",
  "term_id": "GO:0008017"
}